hemocyte development [GO:0007516] (biological process) Also known as: arthropod blood cell development Relationships: is a type of hemopoiesis [GO:0030097]; BFO_0000050 hemocyte differentiation [GO:0042386] Sources: GOC:bf, GOC:mtg_sensu Definition: The process whose specific outcome is the progression of the hemocyte over time, from its formation to the mature structure. Hemocytes are blood cells associated with a hemocoel (the cavity containing most of the major organs of the arthropod body) which are involved in defense and clotting of hemolymph, but not involved in transport of oxygen.